{
  "gene": "UniProtKB:P33527",
  "term_id": "GO:0034775",
  "gene_symbol": "ABCC1",
  "gene_name": "Multidrug resistance-associated protein 1",
  "term_label": "glutathione transmembrane transport"
}